aminoglycan catabolic process [GO:0006026] (biological process) Definition: The chemical reactions and pathways resulting in the breakdown of aminoglycans, any polymer containing amino groups that consists of more than about 10 monosaccharide residues joined to each other by glycosidic linkages. Relationships: is a type of GO:0006022; is a type of macromolecule catabolic process [GO:0009057]; is a type of carbohydrate derivative catabolic process [GO:1901136] Also known as: aminoglycan breakdown, aminoglycan catabolism, aminoglycan degradation Subtypes: GO:0006027, chitin catabolic process [GO:0006032], poly-N-acetyllactosamine catabolic process [GO:0030310] Sources: GOC:ai, ISBN:0198506732